amylopectin catabolic process [GO:2000897] (biological process) Relationships: is a type of GO:0009057; is a type of carbohydrate derivative catabolic process [GO:1901136]; is a type of GO:2000896 Also known as: Amylopectin catabolism Sources: GOC:mengo_curators Definition: The chemical reactions and pathways resulting in the breakdown of an amylopectin. Regulation: regulated by GO:2000945; negatively regulated by negative regulation of amylopectin catabolic process [GO:2000946]; positively regulated by positive regulation of amylopectin catabolic process [GO:2000947]